{
  "term_label": "Unknown cellular component",
  "gene": "UniProtKB:P49918",
  "term_id": "UNKNOWN:0003",
  "gene_name": "Cyclin-dependent kinase inhibitor 1C",
  "gene_symbol": "CDKN1C"
}